{
  "gene": "UniProtKB:Q14318",
  "gene_name": "Peptidyl-prolyl cis-trans isomerase FKBP8",
  "term_id": "GO:0044183",
  "gene_symbol": "FKBP8",
  "term_label": "protein folding chaperone"
}